dADP biosynthetic process [GO:0006173] (biological process) Sources: ISBN:0198506732 Definition: The chemical reactions and pathways resulting in the formation of dADP, deoxyadenosine diphosphate (2'-deoxyadenosine 5'-diphosphate). Also known as: dADP anabolism, dADP biosynthesis, dADP formation, dADP synthesis Relationships: is a type of purine deoxyribonucleotide biosynthetic process [GO:0009153]; is a type of GO:0009183; is a type of GO:0046056